{
  "term_id": "UNKNOWN:0001",
  "term_label": "Unknown molecular function",
  "gene_symbol": "TMEM87B",
  "gene": "UniProtKB:Q96K49",
  "gene_name": "Transmembrane protein 87B"
}